DNA/RNA hybrid annealing activity [GO:0097098] (molecular function) Definition: An activity that facilitates the base-pairing of single-stranded RNA to double-stranded DNA resulting in the formation of R-loops. References: PMID:21699496 Sources: GOC:imk Relationships: is a type of GO:0071667; is a type of annealing activity [GO:0140666]